{
  "term_id": "GO:0045944",
  "gene_symbol": "PPARGC1B",
  "gene": "UniProtKB:Q86YN6",
  "gene_name": "Peroxisome proliferator-activated receptor gamma coactivator 1-beta",
  "term_label": "positive regulation of transcription by RNA polymerase II"
}